{
  "gene": "UniProtKB:Q9Y5M1",
  "term_label": "Unknown biological process",
  "gene_name": "Uncharacterized protein FAM215A",
  "term_id": "UNKNOWN:0002",
  "gene_symbol": "FAM215A"
}